{
  "gene_symbol": "EEF1AKMT3",
  "term_label": "protein-containing complex",
  "gene_name": "EEF1A lysine methyltransferase 3",
  "gene": "UniProtKB:Q96AZ1",
  "term_id": "GO:0032991"
}